{
  "term_id": "GO:0005730",
  "gene": "UniProtKB:Q9BQG0",
  "gene_symbol": "MYBBP1A",
  "gene_name": "Myb-binding protein 1A",
  "term_label": "nucleolus"
}